menaquinone biosynthetic process [GO:0009234] (biological process) Definition: The chemical reactions and pathways resulting in the formation of any of the menaquinones. Structurally, menaquinones consist of a methylated naphthoquinone ring structure and side chains composed of a variable number of unsaturated isoprenoid residues. Menaquinones that have vitamin K activity and are known as vitamin K2. Relationships: is a type of menaquinone metabolic process [GO:0009233]; is a type of ketone biosynthetic process [GO:0042181] References: PMID:6127606 Sources: GOC:jl Also known as: menaquinone anabolism, menaquinone biosynthesis, menaquinone formation, menaquinone synthesis, menatetrenone biosynthesis, menatetrenone biosynthetic process, multiprenylmenaquinone biosynthesis, multiprenylmenaquinone biosynthetic process, vitamin K2 biosynthesis, vitamin K2 biosynthetic process